{
  "term_id": "GO:0005737",
  "gene_symbol": "NEU1",
  "gene_name": "Sialidase-1",
  "gene": "UniProtKB:Q99519",
  "term_label": "cytoplasm"
}